{
  "gene": "UniProtKB:Q9UEE5",
  "gene_symbol": "STK17A",
  "term_label": "nucleus",
  "term_id": "GO:0005634",
  "gene_name": "Serine_threonine-protein kinase 17A"
}